R8 cell fate specification [GO:0045464] (biological process) Definition: The process in which a cell becomes capable of differentiating autonomously into an R8 cell in an environment that is neutral with respect to the developmental pathway; upon specification, the cell fate can be reversed. References: PMID:11880339 Relationships: is_a photoreceptor cell fate specification [GO:0043704]; is part of R8 cell fate commitment [GO:0007460]